{
  "gene": "UniProtKB:Q9NZN5",
  "term_id": "GO:0001664",
  "gene_name": "Rho guanine nucleotide exchange factor 12",
  "term_label": "G protein-coupled receptor binding",
  "gene_symbol": "ARHGEF12"
}